{
  "gene": "UniProtKB:P48058",
  "term_label": "postsynaptic density membrane",
  "gene_symbol": "GRIA4",
  "term_id": "GO:0098839",
  "gene_name": "Glutamate receptor 4"
}